L-cysteine binding [GO:1902485] (molecular function) References: PMID:12941942 Sources: GOC:TermGenie, GOC:bhm Relationships: is a type of amino acid binding [GO:0016597]; is a type of GO:0031406; is a type of cation binding [GO:0043169]; is a type of sulfur compound binding [GO:1901681] Definition: Binding to L-cysteine.